negative regulation of endoplasmic reticulum tubular network organization [GO:1903372] (biological process) References: PMID:24891604 Sources: GOC:TermGenie, GOC:als, GO_REF:0000058 Definition: Any process that stops, prevents or reduces the frequency, rate or extent of endoplasmic reticulum tubular network organization. Relationships: is a type of negative regulation of organelle organization [GO:0010639]; is a type of GO:1903371; negatively regulates endoplasmic reticulum tubular network organization [GO:0071786] Also known as: down regulation of ER tubular network organisation, down regulation of ER tubular network organization, down regulation of endoplasmic reticulum tubular network organisation, down regulation of endoplasmic reticulum tubular network organization, down-regulation of ER tubular network organisation, down-regulation of ER tubular network organization, down-regulation of endoplasmic reticulum tubular network organisation, down-regulation of endoplasmic reticulum tubular network organization, downregulation of ER tubular network organisation, downregulation of ER tubular network organization, downregulation of endoplasmic reticulum tubular network organisation, downregulation of endoplasmic reticulum tubular network organization, negative regulation of ER tubular network organisation, negative regulation of ER tubular network organization, negative regulation of endoplasmic reticulum tubular network organisation, inhibition of ER tubular network organisation, inhibition of ER tubular network organization, inhibition of endoplasmic reticulum tubular network organisation, inhibition of endoplasmic reticulum tubular network organization